glycerol-3-phosphate biosynthetic process [GO:0046167] (biological process) Relationships: is a type of glycerol-3-phosphate metabolic process [GO:0006072]; is a type of GO:0090407; is a type of carbohydrate derivative biosynthetic process [GO:1901137] Definition: The chemical reactions and pathways resulting in the formation of glycerol-3-phosphate, a phosphoric monoester of glycerol. Also known as: glycerol-3-phosphate anabolism, glycerol-3-phosphate biosynthesis, glycerol-3-phosphate formation, glycerol-3-phosphate synthesis Sources: GOC:ai